appressorium-mediated entry into host [GO:0120326] (BP) Relationships: is a type of symbiont entry into host [GO:0044409] References: PMID:14731267, PMID:22589729 Sources: GOC:ach, GOC:krc Definition: Penetration by a symbiont into a host organism via an appressorium. The host is defined as the larger of the organisms involved in a symbiotic interaction. Also known as: appressorium-mediated host invasion, appressorium-mediated host penetration, appressorium-mediated invasion into host, appressorium-mediated penetration into host